{
  "gene_name": "Platelet glycoprotein V",
  "term_id": "GO:1990779",
  "gene_symbol": "GP5",
  "term_label": "glycoprotein Ib-IX-V complex",
  "gene": "UniProtKB:P40197"
}